defense response to symbiont [GO:0140546] (biological process) Sources: GOC:pg Relationships: is a type of defense response to other organism [GO:0098542] Subtypes: GO:0009627, jasmonic acid and ethylene-dependent systemic resistance [GO:0009861], antimicrobial humoral response [GO:0019730], symbiont-induced defense-related programmed cell death [GO:0034050], GO:0045087, killing by host of symbiont cells [GO:0051873], positive regulation of phytoalexin biosynthetic process [GO:0052322], suppression of symbiont entry into host [GO:0052373], GO:0099046, host defense response against symbiont-mediated perturbation of plasma membrane integrity [GO:0140976] Definition: Reactions triggered in response to the presence of a symbiont that act to protect or prevent damage to the host.